{
  "term_label": "ATPase-coupled transmembrane transporter activity",
  "term_id": "GO:0042626",
  "gene_name": "Glucosylceramide transporter ABCA12",
  "gene": "UniProtKB:Q86UK0",
  "gene_symbol": "ABCA12"
}